{
  "gene": "UniProtKB:Q8WVN8",
  "term_id": "GO:0070936",
  "gene_name": "Ubiquitin-conjugating enzyme E2 Q2",
  "gene_symbol": "UBE2Q2",
  "term_label": "protein K48-linked ubiquitination"
}